{
  "gene_name": "GMP synthase [glutamine-hydrolyzing]",
  "gene_symbol": "GMPS",
  "term_id": "GO:0006177",
  "gene": "UniProtKB:P49915",
  "term_label": "GMP biosynthetic process"
}